{
  "term_id": "UNKNOWN:0003",
  "gene_symbol": "CIMAP3",
  "gene_name": "Protein pitchfork",
  "term_label": "Unknown cellular component",
  "gene": "UniProtKB:Q8TCI5"
}